{
  "gene_name": "Ubiquitin carboxyl-terminal hydrolase 46",
  "gene_symbol": "USP46",
  "term_id": "GO:0031647",
  "term_label": "regulation of protein stability",
  "gene": "UniProtKB:P62068"
}